{
  "term_label": "kinetochore",
  "gene_symbol": "SGO1",
  "gene": "UniProtKB:Q5FBB7",
  "term_id": "GO:0000776",
  "gene_name": "Shugoshin 1"
}